{
  "term_label": "cholesterol homeostasis",
  "term_id": "GO:0042632",
  "gene": "UniProtKB:Q9Y5X9",
  "gene_symbol": "LIPG",
  "gene_name": "Endothelial lipase"
}